{
  "gene_symbol": "NEXN",
  "term_id": "GO:0007156",
  "gene": "UniProtKB:Q0ZGT2",
  "term_label": "homophilic cell-cell adhesion",
  "gene_name": "Nexilin"
}